{
  "gene_name": "B2 bradykinin receptor",
  "term_label": "bradykinin receptor activity",
  "gene": "UniProtKB:P30411",
  "term_id": "GO:0004947",
  "gene_symbol": "BDKRB2"
}